{
  "gene_symbol": "WSB2",
  "gene": "UniProtKB:Q9NYS7",
  "term_id": "UNKNOWN:0003",
  "term_label": "Unknown cellular component",
  "gene_name": "WD repeat and SOCS box-containing protein 2"
}